venom-mediated inhibition of low voltage-gated calcium channel activity [GO:0044476] (biological process) Definition: A process in which an organism inhibits or disrupts the activity of a low voltage-gated calcium channel in another organism via the action of a venom. Relationships: is a type of GO:0044474 References: PMID:20920515 Sources: GOC:fj, GOC:jl Also known as: envenomation resulting in negative regulation of low voltage-gated calcium channel activity in another organism, envenomation resulting in negative regulation of low voltage-gated calcium channel activity in other organism